{
  "gene_symbol": "TRMT9B",
  "term_label": "tRNA binding",
  "gene": "UniProtKB:Q9P272",
  "gene_name": "Probable tRNA methyltransferase 9B",
  "term_id": "GO:0000049"
}